phloem loading [GO:0110126] (biological process) Subtypes: phloem sucrose loading [GO:0009915], phloem nitrate loading [GO:0090408], phloem glucosinolate loading [GO:0090449] Definition: The process of loading solutes into the sieve tube or companion cell of the phloem for long distance transport from source to sink. Relationships: is a type of phloem transport [GO:0010233] References: PMID:19025382 Sources: GOC:lr